{
  "term_id": "GO:0045944",
  "term_label": "positive regulation of transcription by RNA polymerase II",
  "gene_name": "Homeobox protein PKNOX1",
  "gene": "UniProtKB:P55347",
  "gene_symbol": "PKNOX1"
}